agmatine aminopropyltransferase activity [GO:0043919] (molecular function) References: PMID:15983049 Sources: RHEA:36487 Definition: Catalysis of the reaction: agmatine + S-adenosyl 3-(methylsulfanyl)propylamine = H+ + N1-(3-aminopropyl)agmatine + S-methyl-5'-thioadenosine. Also known as: agmatine aminopropyl transferase activity Relationships: is a type of GO:0016765